{
  "term_id": "UNKNOWN:0001",
  "gene": "UniProtKB:Q9BXM0",
  "gene_symbol": "PRX",
  "term_label": "Unknown molecular function",
  "gene_name": "Periaxin"
}